{
  "term_id": "UNKNOWN:0003",
  "term_label": "Unknown cellular component",
  "gene": "UniProtKB:P18077",
  "gene_symbol": "RPL35A",
  "gene_name": "Large ribosomal subunit protein eL33"
}